{
  "gene_name": "Cytokine receptor common subunit gamma",
  "gene": "UniProtKB:P31785",
  "term_label": "positive regulation of immunoglobulin production",
  "gene_symbol": "IL2RG",
  "term_id": "GO:0002639"
}